{
  "gene": "UniProtKB:Q9H3H9",
  "gene_name": "Transcription elongation factor A protein-like 2",
  "term_id": "UNKNOWN:0001",
  "gene_symbol": "TCEAL2",
  "term_label": "Unknown molecular function"
}